N-box binding [GO:0071820] (molecular function) References: PMID:11498047 Sources: GOC:yaf Definition: Binding to an N-box, a DNA motif with the consensus sequence CACNAG that is found in the promoters of genes expressed preferentially at synapses. Also known as: N box binding, N-box promoter binding Relationships: is a type of RNA polymerase II cis-regulatory region sequence-specific DNA binding [GO:0000978]